{
  "term_id": "GO:0045944",
  "gene": "UniProtKB:Q96KN3",
  "gene_symbol": "PKNOX2",
  "term_label": "positive regulation of transcription by RNA polymerase II",
  "gene_name": "Homeobox protein PKNOX2"
}